{
  "gene": "UniProtKB:P0DP07",
  "gene_symbol": "IGHV4-31",
  "gene_name": "Immunoglobulin heavy variable 4-31",
  "term_label": "antigen binding",
  "term_id": "GO:0003823"
}